glial cell growth [GO:0042065] (biological process) Subtypes: perineurial glial growth [GO:0042066] Definition: Growth of glial cells, non-neuronal cells that provide support and nutrition, maintain homeostasis, form myelin, and participate in signal transmission in the nervous system. Relationships: is a type of developmental cell growth [GO:0048588]; is part of gliogenesis [GO:0042063] Sources: GOC:dph, GOC:isa_complete, GOC:jid